{
  "term_id": "GO:0042129",
  "gene_symbol": "IL27",
  "gene_name": "Interleukin-27 subunit alpha",
  "gene": "UniProtKB:Q8NEV9",
  "term_label": "regulation of T cell proliferation"
}